{
  "term_label": "homophilic cell-cell adhesion",
  "gene": "UniProtKB:Q96MS0",
  "gene_name": "Roundabout homolog 3",
  "gene_symbol": "ROBO3",
  "term_id": "GO:0007156"
}